{
  "gene_name": "Testis-specific Y-encoded protein 2",
  "term_id": "GO:0000785",
  "term_label": "chromatin",
  "gene": "UniProtKB:A6NKD2",
  "gene_symbol": "TSPY2"
}